{
  "gene_name": "Lysosomal thioesterase PPT2",
  "term_id": "GO:0098599",
  "term_label": "palmitoyl hydrolase activity",
  "gene": "UniProtKB:Q9UMR5",
  "gene_symbol": "PPT2"
}